{
  "term_id": "GO:0000289",
  "gene_name": "Poly(A)-specific ribonuclease PNLDC1",
  "gene": "UniProtKB:Q8NA58",
  "gene_symbol": "PNLDC1",
  "term_label": "nuclear-transcribed mRNA poly(A) tail shortening"
}